{
  "gene_name": "Secretory carrier-associated membrane protein 5",
  "term_id": "GO:0006887",
  "term_label": "exocytosis",
  "gene": "UniProtKB:Q8TAC9",
  "gene_symbol": "SCAMP5"
}